{
  "gene_symbol": "PFN2",
  "term_id": "GO:0032233",
  "term_label": "positive regulation of actin filament bundle assembly",
  "gene_name": "Profilin-2",
  "gene": "UniProtKB:P35080"
}